mitochondrial transcription [GO:0006390] (BP) Relationships: is a type of mitochondrial RNA metabolic process [GO:0000959]; is a type of DNA-templated transcription [GO:0006351]; is part of GO:0140053 Also known as: transcription from mitochondrial promoter References: PMID:23632312 Sources: GOC:jl Regulation: negatively regulated by negative regulation of mitochondrial transcription [GO:0170070]; regulated by GO:1903108; positively regulated by positive regulation of mitochondrial transcription [GO:1903109] Definition: The synthesis of RNA from a mitochondrial DNA template, usually by a specific mitochondrial RNA polymerase.